telomerase holoenzyme complex assembly [GO:1905323] (biological process) Also known as: telomerase holoenzyme complex formation Subtypes: telomerase catalytic core complex assembly [GO:1904868] Definition: The aggregation, arrangement and bonding together of a set of components to form a telomerase holoenzyme complex. References: PMID:26305931 Sources: GOC:TermGenie, GO_REF:0000079 Relationships: is a type of protein-RNA complex assembly [GO:0022618]